{
  "term_label": "cell surface",
  "term_id": "GO:0009986",
  "gene": "UniProtKB:Q5QGT7",
  "gene_symbol": "RTP2",
  "gene_name": "Receptor-transporting protein 2"
}